{
  "term_id": "GO:0005886",
  "gene_name": "V-set and transmembrane domain-containing protein 1",
  "gene_symbol": "VSTM1",
  "gene": "UniProtKB:Q6UX27",
  "term_label": "plasma membrane"
}